{
  "gene_symbol": "TEX28",
  "gene_name": "Testis-specific protein TEX28",
  "term_id": "GO:0012505",
  "gene": "UniProtKB:O15482",
  "term_label": "endomembrane system"
}